metaphase/anaphase transition of cell cycle [GO:0044784] (biological process) Relationships: is a type of regulation of sister chromatid segregation [GO:0033045]; is_a cell cycle phase transition [GO:0044770] Definition: The cell cycle process in which a cell progresses from metaphase to anaphase as part of the cell cycle. Regulation: regulated by GO:1902099; negatively regulated by negative regulation of metaphase/anaphase transition of cell cycle [GO:1902100]; positively regulated by GO:1902101 Subtypes: GO:0007091, metaphase/anaphase transition of meiotic cell cycle [GO:0044785] Sources: GOC:mtg_cell_cycle